{
  "term_id": "GO:0006953",
  "term_label": "acute-phase response",
  "gene_symbol": "CRP",
  "gene": "UniProtKB:P02741",
  "gene_name": "C-reactive protein"
}